{
  "gene_name": "Humanin-like 12",
  "term_id": "UNKNOWN:0003",
  "term_label": "Unknown cellular component",
  "gene": "UniProtKB:P0DMP1",
  "gene_symbol": "MTRNR2L12"
}